{
  "gene_name": "Astrocytic phosphoprotein PEA-15",
  "gene": "UniProtKB:Q15121",
  "term_id": "UNKNOWN:0001",
  "gene_symbol": "PEA15",
  "term_label": "Unknown molecular function"
}